5-lipoxygenase complex [GO:0002180] (CC) Definition: An nuclear membrane protein complex having arachidonate 5-lipoxygenase activity. Relationships: is a type of membrane protein complex [GO:0098796]; is a type of nuclear protein-containing complex [GO:0140513]; is a type of GO:1990204; BFO_0000050 nuclear membrane [GO:0031965] References: PMID:19075240